{
  "term_id": "GO:0005886",
  "gene_name": "Arf-GAP with SH3 domain, ANK repeat and PH domain-containing protein 3",
  "gene": "UniProtKB:Q8TDY4",
  "term_label": "plasma membrane",
  "gene_symbol": "ASAP3"
}